translation termination factor activity [GO:0008079] (molecular function) Definition: Functions in the termination of translation. Sources: GOC:ma Subtypes: translation release factor activity [GO:0003747] Relationships: is a type of translation factor activity [GO:0180051]; is part of translational termination [GO:0006415]